{
  "gene_name": "Fibroblast growth factor 4",
  "term_id": "GO:0043410",
  "gene_symbol": "FGF4",
  "gene": "UniProtKB:P08620",
  "term_label": "positive regulation of MAPK cascade"
}